{
  "gene": "UniProtKB:Q03591",
  "gene_symbol": "CFHR1",
  "term_id": "GO:0005615",
  "term_label": "extracellular space",
  "gene_name": "Complement factor H-related protein 1"
}